{
  "term_id": "UNKNOWN:0001",
  "gene": "UniProtKB:Q9P218",
  "gene_name": "Collagen alpha-1(XX) chain",
  "gene_symbol": "COL20A1",
  "term_label": "Unknown molecular function"
}